{
  "gene_name": "BRISC and BRCA1-A complex member 1",
  "gene": "UniProtKB:Q9NWV8",
  "term_id": "GO:0070552",
  "term_label": "BRISC complex",
  "gene_symbol": "BABAM1"
}